{
  "term_id": "GO:0046580",
  "gene_symbol": "SPRY2",
  "gene_name": "Protein sprouty homolog 2",
  "term_label": "negative regulation of Ras protein signal transduction",
  "gene": "UniProtKB:O43597"
}